{
  "gene_symbol": "RBMY1C",
  "gene": "UniProtKB:P0DJD4",
  "gene_name": "RNA-binding motif protein, Y chromosome, family 1 member C",
  "term_id": "GO:0005681",
  "term_label": "spliceosomal complex"
}